regulation of progesterone secretion [GO:2000870] (biological process) Definition: Any process that modulates the frequency, rate or extent of progesterone secretion. Sources: GOC:sl Relationships: is a type of regulation of female gonad development [GO:2000194]; is a type of regulation of steroid hormone secretion [GO:2000831]; regulates progesterone secretion [GO:0042701] Subtypes: negative regulation of progesterone secretion [GO:2000871], positive regulation of progesterone secretion [GO:2000872]